{
  "term_label": "protein localization to synapse",
  "gene": "UniProtKB:P78352",
  "gene_name": "Disks large homolog 4",
  "term_id": "GO:0035418",
  "gene_symbol": "DLG4"
}